{
  "term_id": "GO:0042448",
  "gene_name": "Aldo-keto reductase family 1 member C3",
  "gene_symbol": "AKR1C3",
  "gene": "UniProtKB:P42330",
  "term_label": "progesterone metabolic process"
}